response to ammonium ion [GO:0060359] (biological process) References: PMID:23509267 Sources: GOC:TermGenie, GO_REF:0000071 Also known as: response to ammonia Subtypes: GO:0071242 Relationships: is a type of response to nitrogen compound [GO:1901698] Definition: Any process that results in a change in state or activity of a cell or an organism (in terms of movement, secretion, enzyme production, gene expression, etc.) as a result of an ammonium stimulus.